{
  "term_id": "GO:0000981",
  "gene": "UniProtKB:Q8NB42",
  "term_label": "DNA-binding transcription factor activity, RNA polymerase II-specific",
  "gene_symbol": "ZNF527",
  "gene_name": "Zinc finger protein 527"
}